{
  "term_id": "GO:0005886",
  "gene_symbol": "EPHB1",
  "gene_name": "Ephrin type-B receptor 1",
  "term_label": "plasma membrane",
  "gene": "UniProtKB:P54762"
}